{
  "term_label": "extracellular space",
  "gene_name": "Putative serine protease 47",
  "term_id": "GO:0005615",
  "gene": "UniProtKB:A8MTI9",
  "gene_symbol": "PRSS47P"
}